{
  "term_label": "chromatin remodeling",
  "gene": "UniProtKB:Q9ULG1",
  "gene_symbol": "INO80",
  "gene_name": "Chromatin-remodeling ATPase INO80",
  "term_id": "GO:0006338"
}